{
  "gene": "UniProtKB:P35237",
  "gene_symbol": "SERPINB6",
  "gene_name": "Serpin B6",
  "term_id": "GO:0005615",
  "term_label": "extracellular space"
}